{
  "term_label": "RNA binding",
  "gene": "UniProtKB:O60231",
  "gene_name": "Pre-mRNA-splicing factor ATP-dependent RNA helicase DHX16",
  "gene_symbol": "DHX16",
  "term_id": "GO:0003723"
}